{
  "gene": "UniProtKB:P23526",
  "term_label": "adenosylhomocysteinase activity",
  "gene_symbol": "AHCY",
  "term_id": "GO:0004013",
  "gene_name": "Adenosylhomocysteinase"
}